dorsal convergence [GO:0060030] (biological process) Definition: The directed migration of individual cells and small groups of cells toward the dorsal midline during gastrulation. This process does not require cell rearrangement. References: PMID:12062082 Sources: GOC:dgf, GOC:dph Relationships: is a type of cell migration involved in gastrulation [GO:0042074]; is part of convergent extension involved in gastrulation [GO:0060027]